{
  "term_id": "GO:0070181",
  "gene": "UniProtKB:P62277",
  "gene_symbol": "RPS13",
  "term_label": "small ribosomal subunit rRNA binding",
  "gene_name": "Small ribosomal subunit protein uS15"
}